{
  "gene": "UniProtKB:Q96BW1",
  "gene_symbol": "UPRT",
  "term_id": "GO:0005737",
  "term_label": "cytoplasm",
  "gene_name": "Uracil phosphoribosyltransferase homolog"
}